{
  "gene_name": "Pseudouridylate synthase PUS7L",
  "term_id": "GO:0001522",
  "term_label": "pseudouridine synthesis",
  "gene_symbol": "PUS7L",
  "gene": "UniProtKB:Q9H0K6"
}